{
  "term_id": "UNKNOWN:0003",
  "gene": "UniProtKB:Q6P9G4",
  "gene_symbol": "TMEM154",
  "gene_name": "Transmembrane protein 154",
  "term_label": "Unknown cellular component"
}